lumenal side of trans-Golgi network membrane [GO:0160282] (cellular component) Also known as: lumenal face of trans-Golgi network membrane, lumenal leaflet of trans-Golgi network membrane, lumenal side of trans-Golgi network References: PMID:23913272, PMID:34597626, PMID:38307322 Definition: The membrane leaflet of the trans-Golgi network membrane that faces the Golgi lumen. Relationships: is a type of GO:0098576; is part of GO:0032588